{
  "term_label": "neuropeptide hormone activity",
  "gene_name": "Pancreatic polypeptide prohormone",
  "term_id": "GO:0005184",
  "gene_symbol": "PPY",
  "gene": "UniProtKB:P01298"
}